atrial cardiac muscle tissue development [GO:0003228] (biological process) Definition: The process whose specific outcome is the progression of cardiac muscle of the atrium over time, from its formation to the mature structure. Sources: GOC:mtg_heart Also known as: atrial myocardium development Relationships: is a type of GO:0048738 Subtypes: sinoatrial node development [GO:0003163]